UV protection [GO:0009650] (biological process) Definition: Any process in which an organism or cell protects itself from ultraviolet radiation (UV), which may also result in resistance to repeated exposure to UV. Also known as: ultraviolet protection, UV resistance, UV tolerance, ultraviolet resistance, ultraviolet tolerance Relationships: is a type of response to UV [GO:0009411] Sources: GOC:jl, GOC:ml